telopode [GO:0120327] (cellular component) Definition: A telopode is a plasma membrane bounded cell projection that is present on a telocyte and is tens to hundreds of microns long. Telopodes form a labyrinthine system communicating through gap junctions. References: PMID:20367664 Sources: GOC:krc, MESH:D000067617 Relationships: is a type of plasma membrane bounded cell projection [GO:0120025]